25-hydroxycholesterol 7-alpha-hydroxylase activity [GO:0033783] (molecular function) Sources: EC:1.14.14.29 Definition: Catalysis of the reactions: 25-hydroxycholesterol + O2 + reduced [NADPH--hemoprotein reductase] = 7alpha,25-dihydroxycholesterol + H+ + H2O + oxidized [NADPH--hemoprotein reductase]. Also converts (25R)-cholest-5-ene-3beta,26-diol to (25R)-cholest-5-en-3beta,7alpha,26-triol. Relationships: is a type of steroid 7-alpha-hydroxylase activity [GO:0008387]; is_a oxidoreductase activity, acting on paired donors, with incorporation or reduction of molecular oxygen, reduced flavin or flavoprotein as one donor, and incorporation of one atom of oxygen [GO:0016712] Also known as: 25-hydroxycholesterol 7alpha-monooxygenase activity, CYP7B1, CYP7B1 oxysterol 7alpha-hydroxylase activity, cholest-5-ene-3beta,25-diol,NADPH:oxygen oxidoreductase (7alpha-hydroxylating) activity